{
  "gene_name": "Protocadherin alpha-13",
  "gene": "UniProtKB:Q9Y5I0",
  "gene_symbol": "PCDHA13",
  "term_id": "GO:0005886",
  "term_label": "plasma membrane"
}